negative regulation of chemokine (C-X-C motif) ligand 1 production [GO:2000339] (biological process) Definition: Any process that stops, prevents or reduces the frequency, rate or extent of chemokine (C-X-C motif) ligand 1 production. Sources: GOC:BHF, GOC:mah Also known as: negative regulation of CXCL1 production, negative regulation of KC production, negative regulation of SCYB1 production, negative regulation of keratinocyte derived chemokine production Relationships: is a type of negative regulation of chemokine production [GO:0032682]; is a type of regulation of chemokine (C-X-C motif) ligand 1 production [GO:2000338]; negatively regulates chemokine (C-X-C motif) ligand 1 production [GO:0072566]